heterotrimeric G-protein binding [GO:0032795] (molecular function) Relationships: is a type of protein-containing complex binding [GO:0044877] Definition: Binding to a heterotrimeric G-protein. Sources: GOC:nln